positive regulation of DNA-templated DNA replication initiation [GO:0032298] (biological process) Subtypes: positive regulation of DNA replication initiation [GO:1903468], positive regulation of initiation of premeiotic DNA replication [GO:1904514] Relationships: is a type of regulation of DNA-templated DNA replication initiation [GO:0030174]; is a type of GO:2000105; positively regulates DNA replication initiation [GO:0006270] Definition: Any process that activates or increases the frequency, rate or extent of initiation of DNA-dependent DNA replication. Also known as: negative regulation of DNA replication initiation, positive regulation of DNA-dependent DNA replication initiation, up regulation of DNA replication initiation, up-regulation of DNA replication initiation, upregulation of DNA replication initiation, activation of DNA replication initiation, stimulation of DNA replication initiation Sources: GOC:mah